{
  "gene_name": "Translation initiation factor IF-2, mitochondrial",
  "term_id": "GO:0005739",
  "gene_symbol": "MTIF2",
  "term_label": "mitochondrion",
  "gene": "UniProtKB:P46199"
}